steroid catabolic process [GO:0006706] (biological process) Definition: The chemical reactions and pathways resulting in the breakdown of steroids, compounds with a 1,2,cyclopentanoperhydrophenanthrene nucleus. Also known as: steroid breakdown, steroid catabolism, steroid degradation Relationships: is a type of steroid metabolic process [GO:0008202]; is a type of lipid catabolic process [GO:0016042] Subtypes: androgen catabolic process [GO:0006710], estrogen catabolic process [GO:0006711], mineralocorticoid catabolic process [GO:0006712], glucocorticoid catabolic process [GO:0006713], C21-steroid hormone catabolic process [GO:0008208], sterol catabolic process [GO:0016127], phytosteroid catabolic process [GO:0016130], vitamin D catabolic process [GO:0042369], ecdysteroid catabolic process [GO:0046344], brexanolone catabolic process [GO:0062175], (17Z)-protosta-17(20),24-dien-3beta-ol catabolic process [GO:1900580], helvolic acid catabolic process [GO:1900811], GO:1904462 Sources: GOC:go_curators